intermediate filament depolymerization [GO:0045106] (BP) Definition: Disassembly of intermediate filaments by the removal of component monomers from a filament. Relationships: is a type of intermediate filament polymerization or depolymerization [GO:0045105]; is a type of GO:0051261 Sources: GOC:mah, ISBN:0716731363 Regulation: RO_0002211 by regulation of intermediate filament depolymerization [GO:0030842]; negatively regulated by negative regulation of intermediate filament depolymerization [GO:0030843]; positively regulated by positive regulation of intermediate filament depolymerization [GO:0030844]